acinar cell differentiation involved in salivary gland development [GO:0060704] (BP) Sources: GOC:dph, GOC:tb Definition: The process in which a relatively unspecialized cell acquires specialized structural and/or functional features that characterize an acinar cell of the salivary gland. Acinar cells are protein-secreting cells in the gland. Relationships: is a type of GO:0060690; is a type of GO:0090425